{
  "term_id": "GO:0000981",
  "gene_name": "Protein odd-skipped-related 1",
  "gene": "UniProtKB:Q8TAX0",
  "gene_symbol": "OSR1",
  "term_label": "DNA-binding transcription factor activity, RNA polymerase II-specific"
}